{
  "gene_symbol": "RRP8",
  "gene_name": "Ribosomal RNA-processing protein 8",
  "term_label": "nucleolus",
  "gene": "UniProtKB:O43159",
  "term_id": "GO:0005730"
}